diphosphate-protein phosphotransferase activity [GO:0047321] (molecular function) Sources: EC:2.7.99.1, MetaCyc:2.7.99.1-RXN Also known as: diphosphate:microsomal-membrane-protein O-phosphotransferase activity, DiPPT, pyrophosphate-protein phosphotransferase activity, pyrophosphate:protein phosphotransferase activity, triphosphate-protein phosphotransferase activity, triphosphate:microsomal-membrane-protein phosphotransferase activity Relationships: is a type of kinase activity [GO:0016301]; is a type of GO:0016773 Definition: Catalysis of the reaction: microsomal-membrane protein + diphosphate = diphosphate + O-phospho-microsomal-membrane protein.